{
  "gene": "UniProtKB:Q6DN90",
  "term_id": "GO:0098839",
  "term_label": "postsynaptic density membrane",
  "gene_symbol": "IQSEC1",
  "gene_name": "IQ motif and SEC7 domain-containing protein 1"
}